{
  "term_label": "positive regulation of adherens junction organization",
  "gene_symbol": "ADD1",
  "term_id": "GO:1903393",
  "gene": "UniProtKB:P35611",
  "gene_name": "Alpha-adducin"
}